{
  "term_label": "regulation of cell population proliferation",
  "term_id": "GO:0042127",
  "gene_name": "Signal transducer and activator of transcription 4",
  "gene": "UniProtKB:Q14765",
  "gene_symbol": "STAT4"
}